{
  "term_id": "GO:0001042",
  "gene_symbol": "RRN3",
  "gene": "UniProtKB:Q9NYV6",
  "term_label": "RNA polymerase I core binding",
  "gene_name": "RNA polymerase I-specific transcription initiation factor RRN3"
}